{
  "gene_name": "Calmodulin-regulated spectrin-associated protein 2",
  "term_label": "negative regulation of microtubule depolymerization",
  "gene": "UniProtKB:Q08AD1",
  "term_id": "GO:0007026",
  "gene_symbol": "CAMSAP2"
}